regulation of establishment of cell polarity regulating cell shape [GO:2000782] (biological process) Definition: Any process that modulates the frequency, rate or extent of establishment of cell polarity regulating cell shape. Sources: GOC:Mah Subtypes: GO:2000783, GO:2000784 Relationships: is_a regulation of establishment of cell polarity [GO:2000114]; is a type of regulation of establishment or maintenance of cell polarity regulating cell shape [GO:2000769]; regulates GO:0071964